{
  "gene": "UniProtKB:Q6UW78",
  "term_id": "GO:0005743",
  "gene_symbol": "UQCC3",
  "term_label": "mitochondrial inner membrane",
  "gene_name": "Ubiquinol-cytochrome-c reductase complex assembly factor 3"
}